polyketide synthase complex [GO:0034081] (cellular component) Definition: A protein complex that carries out enzymatic reactions involved in the biosynthesis of polyketides, any of a diverse group of natural products synthesized via linear poly-beta-ketones. Relationships: is_a GO:1902494; is part of cytoplasm [GO:0005737] References: PMID:12636085 Sources: GOC:mah Subtypes: GO:0034082, type III polyketide synthase complex [GO:0034083] Also known as: PKS complex, PKS